{
  "term_id": "UNKNOWN:0002",
  "gene": "UniProtKB:Q8WY22",
  "gene_symbol": "BRI3BP",
  "gene_name": "BRI3-binding protein",
  "term_label": "Unknown biological process"
}